regulation of receptor clustering [GO:1903909] (biological process) Subtypes: regulation of glutamate receptor clustering [GO:0106104], GO:1903910, GO:1903911, regulation of skeletal muscle acetylcholine-gated channel clustering [GO:1904393] Relationships: is a type of regulation of protein localization to membrane [GO:1905475]; regulates receptor clustering [GO:0043113] References: PMID:23575248 Sources: GOC:TermGenie, GOC:als, GO_REF:0000058 Definition: Any process that modulates the frequency, rate or extent of receptor clustering.